{
  "gene_name": "T cell receptor alpha variable 3",
  "gene": "UniProtKB:A0A0B4J244",
  "term_id": "UNKNOWN:0001",
  "gene_symbol": "TRAV3",
  "term_label": "Unknown molecular function"
}